{
  "term_label": "Unknown cellular component",
  "term_id": "UNKNOWN:0003",
  "gene_symbol": "TNP2",
  "gene": "UniProtKB:Q05952",
  "gene_name": "Nuclear transition protein 2"
}